{
  "gene": "UniProtKB:Q96KG9",
  "term_label": "Unknown molecular function",
  "term_id": "UNKNOWN:0001",
  "gene_name": "N-terminal kinase-like protein",
  "gene_symbol": "SCYL1"
}